{
  "term_id": "GO:0005737",
  "gene_symbol": "CDKN2A",
  "term_label": "cytoplasm",
  "gene_name": "Cyclin-dependent kinase inhibitor 2A",
  "gene": "UniProtKB:P42771"
}